{
  "gene_name": "Histone PARylation factor 1",
  "term_label": "double-strand break repair",
  "gene_symbol": "HPF1",
  "term_id": "GO:0006302",
  "gene": "UniProtKB:Q9NWY4"
}